{
  "gene_symbol": "SLC36A4",
  "gene": "UniProtKB:Q6YBV0",
  "term_label": "L-alanine transmembrane transporter activity",
  "term_id": "GO:0015180",
  "gene_name": "Neutral amino acid uniporter 4"
}